{
  "term_label": "SUMO binding",
  "term_id": "GO:0032183",
  "gene_symbol": "CBX4",
  "gene_name": "E3 SUMO-protein ligase CBX4",
  "gene": "UniProtKB:O00257"
}